{
  "gene_name": "Protein PBDC1",
  "term_label": "protein folding chaperone",
  "gene_symbol": "PBDC1",
  "gene": "UniProtKB:Q9BVG4",
  "term_id": "GO:0044183"
}